{
  "gene_name": "Uncharacterized protein C2orf80",
  "term_id": "UNKNOWN:0001",
  "gene_symbol": "C2orf80",
  "gene": "UniProtKB:Q0P641",
  "term_label": "Unknown molecular function"
}